{
  "gene": "UniProtKB:O43159",
  "term_label": "regulation of transcription by glucose",
  "gene_name": "Ribosomal RNA-processing protein 8",
  "gene_symbol": "RRP8",
  "term_id": "GO:0046015"
}